{
  "gene_name": "Leucine-rich repeat-containing protein 61",
  "term_id": "UNKNOWN:0003",
  "gene_symbol": "LRRC61",
  "term_label": "Unknown cellular component",
  "gene": "UniProtKB:Q9BV99"
}